peptidyl-L-cysteine S-palmitoylation [GO:0018230] (biological process) Sources: RESID:AA0106 Note: Palmitoylation of a non-terminal cysteine residue always occurs on a sulfur (S) atom. Regulation: regulated by regulation of peptidyl-L-cysteine S-palmitoylation [GO:1902662]; negatively regulated by negative regulation of peptidyl-L-cysteine S-palmitoylation [GO:1902663]; positively regulated by positive regulation of peptidyl-L-cysteine S-palmitoylation [GO:1902664] Definition: The covalent attachment of a palmitoyl group to a sulfur (S) atom within a cysteine residue to form peptidyl-S-palmitoyl-L-cysteine. Also known as: peptidyl-S-palmitoyl-L-cysteine anabolism from peptidyl-cysteine, peptidyl-S-palmitoyl-L-cysteine biosynthetic process from peptidyl-cysteine, peptidyl-S-palmitoyl-L-cysteine formation from peptidyl-cysteine, peptidyl-S-palmitoyl-L-cysteine synthesis from peptidyl-cysteine, peptidyl-cysteine S-palmitoylation Relationships: is a type of GO:0018231; is_a protein palmitoylation [GO:0018345]